{
  "gene_name": "Secreted and transmembrane protein 1",
  "term_label": "Unknown biological process",
  "term_id": "UNKNOWN:0002",
  "gene_symbol": "SECTM1",
  "gene": "UniProtKB:Q8WVN6"
}